{
  "term_id": "UNKNOWN:0002",
  "gene_symbol": "LRRC51",
  "gene": "UniProtKB:Q96E66",
  "term_label": "Unknown biological process",
  "gene_name": "Leucine-rich repeat-containing protein 51"
}